{
  "term_id": "GO:0007160",
  "gene_symbol": "CD34",
  "term_label": "cell-matrix adhesion",
  "gene": "UniProtKB:P28906",
  "gene_name": "Hematopoietic progenitor cell antigen CD34"
}